integrator complex assembly [GO:0160234] (biological process) Relationships: is a type of protein-containing complex assembly [GO:0065003] Definition: The aggregation, arrangement and bonding together of a set of components to form the integrator complex. References: PMID:39032489, PMID:39032490